determination of dorsal identity [GO:0048263] (biological process) Also known as: determination of adaxial identity Definition: Determination of the identity of part of an organism or organ where those parts are of the type that occur in the dorsal region. Identity is considered to be the aggregate of characteristics by which a structure is recognized. Regulation: regulated by GO:2000015; negatively regulated by negative regulation of determination of dorsal identity [GO:2000016]; positively regulated by GO:2000017 Sources: GOC:jid Relationships: is a type of dorsal/ventral pattern formation [GO:0009953]; is part of determination of dorsal/ventral asymmetry [GO:0048262]